{
  "term_id": "GO:0045296",
  "gene_symbol": "CDH18",
  "gene_name": "Cadherin-18",
  "gene": "UniProtKB:Q13634",
  "term_label": "cadherin binding"
}